{
  "gene_name": "CTP synthase 1",
  "gene": "UniProtKB:P17812",
  "gene_symbol": "CTPS1",
  "term_id": "GO:0005737",
  "term_label": "cytoplasm"
}